spindle matrix [GO:1990047] (CC) Definition: A proteinaceous, nuclear-derived structure that embeds the microtubule spindle apparatus from pole to pole in a microtubule-independent manner during mitosis. References: PMID:19273613, PMID:22855526 Sources: GOC:ans Relationships: is a type of cellular anatomical structure [GO:0110165]; is part of cytoskeleton [GO:0005856]